embryo sac development [GO:0009553] (biological process) Sources: GOC:mtg_plant, GOC:tb Also known as: female gametophyte development Relationships: is a type of gametophyte development [GO:0048229] Definition: The process whose specific outcome is the progression of the embryo sac over time, from its formation to the mature structure. The process begins with the meiosis of the megasporocyte to form four haploid megaspores. Three of the megaspores disintegrate, and the fourth undergoes mitosis giving rise to a binucleate syncytial embryo sac. The two haploid nuclei migrate to the opposite poles of the embryo sac and then undergo two rounds of mitosis generating four haploid nuclei at each pole. One nucleus from each set of four migrates to the center of the cell. Cellularization occurs, resulting in an eight-nucleate seven-celled structure. This structure contains two synergid cells and an egg cell at the micropylar end, and three antipodal cells at the other end. A binucleate endosperm mother cell is formed at the center. The two polar nuclei fuse resulting in a mononucleate diploid endosperm mother cell. The three antipodal cells degenerate.